neural crest cell delamination [GO:0036032] (biological process) Subtypes: cardiac neural crest cell delamination [GO:0036036] Relationships: is_a delamination [GO:0060232] Definition: The negative regulation of cell adhesion process in which a neural crest cell physically separates from the rest of the neural tube. References: PMID:17076275 Sources: CL:0000333 Also known as: neural crest cell emigration, neural crest cell individualization, neural crest cell segregation